{
  "term_id": "UNKNOWN:0001",
  "gene": "UniProtKB:A0A494C103",
  "term_label": "Unknown molecular function",
  "gene_name": "CUB domain-containing protein",
  "gene_symbol": "SPADH"
}